branching involved in open tracheal system development [GO:0060446] (BP) Sources: GOC:dph Relationships: is a type of GO:0048754; is part of GO:0007424 Definition: The process in which the anatomical structures of branches in the open tracheal system are generated and organized. Subtypes: primary branching, open tracheal system [GO:0007428], secondary branching, open tracheal system [GO:0007429], GO:0007430